{
  "term_id": "UNKNOWN:0001",
  "term_label": "Unknown molecular function",
  "gene": "UniProtKB:O14526",
  "gene_symbol": "FCHO1",
  "gene_name": "F-BAR domain only protein 1"
}